homotetrameric ADPG pyrophosphorylase complex [GO:0030930] (cellular component) Definition: A protein complex composed of four identical subunits that possesses ADPG pyrophosphorylase activity. Examples of this component are found in Bacterial species. Sources: GOC:mah, GOC:mtg_sensu Relationships: is a type of GO:0030929